ribonucleotide biosynthetic process [GO:0009260] (biological process) Sources: GOC:go_curators, ISBN:0198506732 Subtypes: purine ribonucleotide biosynthetic process [GO:0009152], pyrimidine ribonucleotide biosynthetic process [GO:0009220], FMN biosynthetic process [GO:0009398], GO:0120232 Also known as: ribonucleotide anabolism, ribonucleotide biosynthesis, ribonucleotide formation, ribonucleotide synthesis Relationships: is a type of GO:0009165; is a type of GO:0009259; is a type of ribose phosphate biosynthetic process [GO:0046390] Definition: The chemical reactions and pathways resulting in the formation of a ribonucleotide, a compound consisting of ribonucleoside (a base linked to a ribose sugar) esterified with a phosphate group at either the 3' or 5'-hydroxyl group of the sugar.